{
  "gene": "UniProtKB:Q6U736",
  "term_label": "plasma membrane",
  "gene_symbol": "OPN5",
  "gene_name": "Opsin-5",
  "term_id": "GO:0005886"
}